female germline ring canal formation [GO:0007301] (biological process) Definition: Assembly of the intercellular bridges that connect the germ-line cells of a female cyst. Also known as: nurse cell ring canal formation, ovarian ring canal formation Sources: ISBN:0879694238 Relationships: is a type of germline ring canal formation [GO:0030725]; is part of germarium-derived egg chamber formation [GO:0007293]; is part of ovarian nurse cell to oocyte transport [GO:0007300]